{
  "gene_symbol": "SLC25A36",
  "gene": "UniProtKB:Q96CQ1",
  "gene_name": "Solute carrier family 25 member 36",
  "term_label": "pyrimidine nucleotide transmembrane transporter activity",
  "term_id": "GO:0015218"
}